{
  "term_id": "GO:0036297",
  "gene_symbol": "HMCES",
  "gene_name": "Abasic site processing protein HMCES",
  "gene": "UniProtKB:Q96FZ2",
  "term_label": "interstrand cross-link repair"
}